{
  "gene_symbol": "CHGA",
  "gene": "UniProtKB:P10645",
  "gene_name": "Chromogranin-A",
  "term_id": "GO:0042583",
  "term_label": "chromaffin granule"
}